{
  "gene_name": "Junctional adhesion molecule-like",
  "term_id": "GO:0005886",
  "gene": "UniProtKB:Q86YT9",
  "term_label": "plasma membrane",
  "gene_symbol": "JAML"
}